{
  "gene": "UniProtKB:A0A075B6W3",
  "term_label": "Unknown cellular component",
  "term_id": "UNKNOWN:0003",
  "gene_name": "T cell receptor alpha joining 33 (Fragment)",
  "gene_symbol": "TRAJ33"
}